{
  "gene": "UniProtKB:P40879",
  "term_id": "GO:0005886",
  "gene_symbol": "SLC26A3",
  "gene_name": "Chloride anion exchanger",
  "term_label": "plasma membrane"
}